{
  "gene_name": "Coatomer subunit zeta-2",
  "term_label": "intra-Golgi vesicle-mediated transport",
  "gene": "UniProtKB:Q9P299",
  "term_id": "GO:0006891",
  "gene_symbol": "COPZ2"
}